{
  "term_label": "cytoplasm",
  "gene_symbol": "MIB2",
  "term_id": "GO:0005737",
  "gene_name": "E3 ubiquitin-protein ligase MIB2",
  "gene": "UniProtKB:Q96AX9"
}